proteasome storage granule [GO:0034515] (cellular component) Definition: An aggregation of proteasome core protease (CP) and regulatory particle (RP) complexes that localizes in the cytoplasm as dot-like structures when cells are in a quiescent state. Relationships: is_a intracellular membraneless organelle [GO:0043232]; is part of GO:0005737 Also known as: PSG References: PMID:18504300, PMID:30204036 Sources: GOC:krc, GOC:rb